{
  "gene": "UniProtKB:Q9UIG0",
  "gene_name": "Tyrosine-protein kinase BAZ1B",
  "term_label": "histone kinase activity",
  "gene_symbol": "BAZ1B",
  "term_id": "GO:0035173"
}